{
  "gene": "UniProtKB:P84098",
  "term_label": "Unknown biological process",
  "gene_symbol": "RPL19",
  "gene_name": "Large ribosomal subunit protein eL19",
  "term_id": "UNKNOWN:0002"
}